epithelium migration [GO:0090132] (biological process) Sources: GOC:ascb_2009, GOC:dph, GOC:tb Definition: The process in which the population of cells that make up an epithelium undergo directed movement. Relationships: is a type of tissue migration [GO:0090130] Subtypes: GO:0090133, epithelium migration involved in imaginal disc-derived wing morphogenesis [GO:0090252]